{
  "gene_name": "Immunoglobulin lambda variable 7-46",
  "term_id": "GO:0019814",
  "term_label": "immunoglobulin complex",
  "gene_symbol": "IGLV7-46",
  "gene": "UniProtKB:A0A075B6I9"
}